regulation of behavioral fear response [GO:2000822] (biological process) Sources: GOC:BHF Definition: Any process that modulates the frequency, rate or extent of behavioral fear response. Relationships: is a type of regulation of defense response [GO:0031347]; is a type of GO:0050795; is a type of regulation of fear response [GO:1903365]; regulates behavioral fear response [GO:0001662] Subtypes: negative regulation of behavioral fear response [GO:2000986], positive regulation of behavioral fear response [GO:2000987] Also known as: regulation of behavioural fear response